2-aminoadipate transaminase activity [GO:0047536] (molecular function) Definition: Catalysis of the reaction: 2-oxoglutarate + L-2-aminoadipate = 2-oxoadipate + L-glutamate. Also known as: 2-aminoadipate aminotransferase activity, 2-aminoadipic aminotransferase activity, L-2-aminoadipate:2-oxoglutarate aminotransferase activity, alpha-aminoadipate aminotransferase activity, glutamate-alpha-ketoadipate transaminase activity, glutamic-ketoadipic transaminase activity Sources: EC:2.6.1.39, RHEA:12601 Relationships: is a type of GO:0008483